{
  "term_label": "rRNA binding",
  "term_id": "GO:0019843",
  "gene_symbol": "PTCD3",
  "gene": "UniProtKB:Q96EY7",
  "gene_name": "Small ribosomal subunit protein mS39"
}